{
  "gene_symbol": "POP4",
  "term_id": "GO:0000172",
  "term_label": "ribonuclease MRP complex",
  "gene": "UniProtKB:O95707",
  "gene_name": "Ribonuclease P protein subunit p29"
}